T cell receptor V(D)J recombination [GO:0033153] (BP) Sources: GOC:add, ISBN:0781700221 Definition: The process in which T cell receptor V, D, and J, or V and J gene segments, depending on the specific locus, are recombined within a single locus utilizing the conserved heptamer and nonomer recombination signal sequences (RSS). Also known as: T cell receptor V(D)J joining, T-cell receptor V(D)J recombination, TCR V(D)J recombination, T cell receptor V-D-J joining, T cell receptor V-D-J recombination, T cell receptor V-J joining, T cell receptor V-J recombination Relationships: is a type of somatic recombination of T cell receptor gene segments [GO:0002681]; is a type of GO:0033151